{
  "term_id": "GO:0005829",
  "gene_symbol": "ZC3H15",
  "gene": "UniProtKB:Q8WU90",
  "gene_name": "Zinc finger CCCH domain-containing protein 15",
  "term_label": "cytosol"
}